{
  "term_id": "GO:0016514",
  "gene_symbol": "SMARCD3",
  "gene": "UniProtKB:Q6STE5",
  "term_label": "SWI/SNF complex",
  "gene_name": "SWI_SNF-related matrix-associated actin-dependent regulator of chromatin subfamily D member 3"
}